positive regulation of vesicle fusion with Golgi apparatus [GO:0106216] (biological process) Definition: Any process that activates or increases the frequency, rate or extent of vesicle fusion with Golgi apparatus. Relationships: is a type of positive regulation of vesicle fusion [GO:0031340]; is a type of regulation of vesicle fusion with Golgi apparatus [GO:0106214]; RO_0002213 vesicle fusion with Golgi apparatus [GO:0048280] References: PMID:26195667 Sources: GOC:se